regulation of entry of bacterium into host cell [GO:2000535] (biological process) Definition: Any process that modulates the frequency, rate or extent of entry of bacterium into host cell. Relationships: is a type of modulation by symbiont of entry into host [GO:0052372]; RO_0002211 GO:0035635 Sources: GOC:obol Subtypes: negative regulation of entry of bacterium into host cell [GO:2000536] Also known as: regulation of bacterial entry into host cell, regulation of invasion of bacteria into host cell